{
  "term_id": "UNKNOWN:0003",
  "gene_symbol": "IKZF3",
  "term_label": "Unknown cellular component",
  "gene_name": "Zinc finger protein Aiolos",
  "gene": "UniProtKB:Q9UKT9"
}